{
  "term_id": "UNKNOWN:0003",
  "term_label": "Unknown cellular component",
  "gene_symbol": "FAM204A",
  "gene": "UniProtKB:Q9H8W3",
  "gene_name": "Protein FAM204A"
}